{
  "gene_symbol": "ZNF705G",
  "gene_name": "Putative zinc finger protein 705G",
  "term_id": "GO:0006357",
  "term_label": "regulation of transcription by RNA polymerase II",
  "gene": "UniProtKB:A8MUZ8"
}